heterochromatin domain [GO:1990343] (CC) Definition: A region of heterochromatin that is formed dynamically under specific growth conditions by a process that requires RNAi, and is enriched in histone H3 methylated on lysine 9 (H3K9me). References: PMID:23151475, PMID:24210919 Also known as: HOOD Note: An example of this type of heterochromatin is found in Schizosaccharomyces pombe, where heterochromatin domains preferentially assemble at sexual differentiation genes and retrotransposons. Relationships: is a type of GO:0000792